peroxisomal transport [GO:0043574] (biological process) Definition: Transport of substances into, out of or within a peroxisome, a small, membrane-bounded organelle that uses dioxygen (O2) to oxidize organic molecules. Sources: GOC:jl Relationships: is a type of intracellular transport [GO:0046907] Subtypes: GO:0015919